fructosamine biosynthetic process [GO:0030391] (biological process) Subtypes: fructoselysine biosynthetic process [GO:1901282] Sources: GOC:jl, ISBN:0192801023 Relationships: is a type of GO:0030389; is a type of amino sugar biosynthetic process [GO:0046349] Also known as: fructosamine anabolism, fructosamine biosynthesis, fructosamine formation, fructosamine synthesis Definition: The chemical reactions and pathways resulting in the formation of fructosamine, a fructose molecule containing an amino group in place of a hydroxyl group.